proepicardium development [GO:0003342] (biological process) Definition: The progression of the proepicardium from its formation to the mature structure. The proepicardium is an outpouching of the septum transversum. References: PMID:18722343 Sources: GOC:dph Relationships: is a type of mesenchyme development [GO:0060485]; is part of septum transversum development [GO:0003343]